{
  "gene_symbol": "HS2ST1",
  "gene": "UniProtKB:Q7LGA3",
  "gene_name": "Heparan sulfate 2-O-sulfotransferase 1",
  "term_label": "Unknown cellular component",
  "term_id": "UNKNOWN:0003"
}